hemidesmosome associated protein complex [GO:0098733] (cellular component) Definition: Any protein complex that is part of or has some part in a hemidesmosome. Relationships: is a type of GO:0032991 Sources: GOC:dos